{
  "gene_name": "Olfactory receptor",
  "gene": "UniProtKB:A0A2R8YEG4",
  "gene_symbol": "OR2A1",
  "term_id": "UNKNOWN:0001",
  "term_label": "Unknown molecular function"
}